{
  "gene": "UniProtKB:Q6NUN9",
  "gene_name": "Zinc finger protein 746",
  "term_id": "GO:0005634",
  "gene_symbol": "ZNF746",
  "term_label": "nucleus"
}